{
  "gene_name": "Gap junction alpha-9 protein",
  "gene_symbol": "GJA9",
  "term_id": "GO:0005922",
  "term_label": "connexin complex",
  "gene": "UniProtKB:P57773"
}